{
  "gene_symbol": "COPS6",
  "gene": "UniProtKB:Q7L5N1",
  "term_label": "Unknown biological process",
  "gene_name": "COP9 signalosome complex subunit 6",
  "term_id": "UNKNOWN:0002"
}